{
  "term_label": "late endosome",
  "gene": "UniProtKB:Q8IZ07",
  "gene_name": "Ankyrin repeat domain-containing protein 13A",
  "gene_symbol": "ANKRD13A",
  "term_id": "GO:0005770"
}